ommatidial rotation [GO:0016318] (biological process) Relationships: is_a GO:0007389; is part of GO:0042067 References: PMID:10725247 Definition: The process in which photoreceptors are arranged in ommatidia in the dorsal and ventral fields to be mirror images. The polarity is established in the imaginal discs concurrently with cell fate specification.